{
  "gene_symbol": "CD300LD-AS1",
  "term_label": "Unknown cellular component",
  "term_id": "UNKNOWN:0003",
  "gene": "UniProtKB:Q96MU5",
  "gene_name": "Uncharacterized protein CD300LD-AS1"
}